{
  "gene_symbol": "RAB2B",
  "term_id": "GO:0016192",
  "gene_name": "Ras-related protein Rab-2B",
  "gene": "UniProtKB:Q8WUD1",
  "term_label": "vesicle-mediated transport"
}